secondary active p-aminobenzoyl-glutamate transmembrane transporter activity [GO:0015558] (MF) Definition: Enables the transfer of p-aminobenzoyl-glutamate from one side of a membrane to the other, up its concentration gradient. The transporter binds the solute and undergoes a series of conformational changes. Transport works equally well in either direction and is driven by a chemiosmotic source of energy. Secondary active transporters include symporters and antiporters. p-aminobenzoyl-glutamate is the anion of p-aminobenzoyl-glutamic acid. Relationships: is_a GO:0005310; is a type of secondary active transmembrane transporter activity [GO:0015291]; is a type of dipeptide transmembrane transporter activity [GO:0071916]; is a type of modified amino acid transmembrane transporter activity [GO:0072349] Sources: GOC:ai Also known as: p-aminobenzoyl-glutamate transmembrane transporter activity, p-aminobenzoyl-glutamate transporter activity, p-aminobenzoyl-glutamate uptake permease activity, p-aminobenzoyl-glutamate uptake transmembrane transporter activity